{
  "term_label": "glucose-1,6-bisphosphate synthase activity",
  "gene": "UniProtKB:Q6PCE3",
  "gene_name": "Glucose 1,6-bisphosphate synthase",
  "term_id": "GO:0047933",
  "gene_symbol": "PGM2L1"
}